(S)-carnitine 3-dehydrogenase activity [GO:0047041] (molecular function) Relationships: is a type of oxidoreductase activity, acting on the CH-OH group of donors, NAD or NADP as acceptor [GO:0016616] Sources: EC:1.1.1.254, RHEA:11556 Also known as: (S)-carnitine:NAD+ oxidoreductase activity, D-carnitine dehydrogenase activity Definition: Catalysis of the reaction: (S)-carnitine + NAD+ = 3-dehydrocarnitine + H+ + NADH.